type 1 melanin-concentrating hormone receptor binding [GO:0031777] (molecular function) Relationships: is a type of GO:0031776 Also known as: type 1 melanin-concentrating hormone receptor ligand Definition: Binding to a type 1 melanin-concentrating hormone receptor. Sources: GOC:mah, GOC:nln